{
  "gene_symbol": "PWP2",
  "term_id": "GO:0000462",
  "gene_name": "Periodic tryptophan protein 2 homolog",
  "term_label": "maturation of SSU-rRNA from tricistronic rRNA transcript (SSU-rRNA, 5.8S rRNA, LSU-rRNA)",
  "gene": "UniProtKB:Q15269"
}